{
  "gene_name": "Olfactory receptor 9G4",
  "term_id": "GO:0004984",
  "term_label": "olfactory receptor activity",
  "gene": "UniProtKB:Q8NGQ1",
  "gene_symbol": "OR9G4"
}